{
  "term_label": "Unknown biological process",
  "term_id": "UNKNOWN:0002",
  "gene_name": "Mammalian ependymin-related protein 1",
  "gene": "UniProtKB:Q9UM22",
  "gene_symbol": "EPDR1"
}